{
  "gene_symbol": "SLC51A",
  "gene_name": "Organic solute transporter subunit alpha",
  "gene": "UniProtKB:Q86UW1",
  "term_label": "bile acid and bile salt transport",
  "term_id": "GO:0015721"
}